{
  "term_label": "regulation of transcription by RNA polymerase II",
  "gene_name": "Transcription factor Sp5",
  "gene_symbol": "SP5",
  "gene": "UniProtKB:Q6BEB4",
  "term_id": "GO:0006357"
}